{
  "term_id": "GO:0004972",
  "gene_symbol": "GRIN2A",
  "term_label": "NMDA glutamate receptor activity",
  "gene": "UniProtKB:Q12879",
  "gene_name": "Glutamate receptor ionotropic, NMDA 2A"
}